{
  "gene_symbol": "MC3R",
  "gene_name": "Melanocortin receptor 3",
  "term_label": "peptide hormone binding",
  "term_id": "GO:0017046",
  "gene": "UniProtKB:P41968"
}